hopanoid catabolic process [GO:0019743] (biological process) Relationships: is a type of triterpenoid catabolic process [GO:0016105] Sources: ISBN:0198547684 Definition: The chemical reactions and pathways resulting in the breakdown of hopanoids, pentacyclic sterol-like compounds based on the hopane nucleus. Also known as: hopanoid breakdown, hopanoid catabolism, hopanoid degradation